{
  "gene_name": "Quinone oxidoreductase-like protein 1",
  "term_label": "Unknown molecular function",
  "term_id": "UNKNOWN:0001",
  "gene_symbol": "CRYZL1",
  "gene": "UniProtKB:O95825"
}